G-protein gamma-subunit binding [GO:0031682] (MF) Definition: Binding to a G-protein gamma subunit. Sources: GOC:mah Also known as: G-gamma protein subunit binding Relationships: is a type of protein binding [GO:0005515]